antigen processing and presentation of exogenous peptide antigen via MHC class Ib [GO:0002477] (biological process) Relationships: is a type of antigen processing and presentation of peptide antigen via MHC class Ib [GO:0002428]; is a type of antigen processing and presentation of exogenous peptide antigen [GO:0002478] Subtypes: antigen processing and presentation of exogenous protein antigen via MHC class Ib, TAP-dependent [GO:0002481], antigen processing and presentation of exogenous protein antigen via MHC class Ib, TAP-independent [GO:0002482] References: PMID:15928678 Sources: GOC:add Also known as: exogenous peptide antigen processing and presentation via MHC class Ib Definition: The process in which an antigen-presenting cell expresses a peptide antigen of exogenous origin on its cell surface in association with an MHC class Ib protein complex. The peptide is typically a fragment of a larger exogenous protein which has been degraded within the cell. Class Ib here refers to non-classical class I molecules, such as those of the HLA-E gene family.